negative regulation of t-circle formation [GO:1904430] (biological process) Definition: Any process that stops, prevents or reduces the frequency, rate or extent of t-circle formation. Also known as: down regulation of t-circle formation, down regulation of telomeric circle formation, down-regulation of t-circle formation, down-regulation of telomeric circle formation, downregulation of t-circle formation, downregulation of telomeric circle formation, negative regulation of telomeric circle formation, inhibition of t-circle formation, inhibition of telomeric circle formation Relationships: is a type of GO:0051053; is a type of negative regulation of cellular component organization [GO:0051129]; is a type of regulation of t-circle formation [GO:1904429]; negatively regulates t-circle formation [GO:0090656] References: PMID:22579284 Sources: GOC:BHF, GOC:BHF_telomere, GOC:TermGenie, GOC:nc, GO_REF:0000058